{
  "term_label": "Unknown biological process",
  "term_id": "UNKNOWN:0002",
  "gene_name": "Interleukin-17 receptor C",
  "gene": "UniProtKB:Q8NAC3",
  "gene_symbol": "IL17RC"
}